{
  "term_id": "UNKNOWN:0001",
  "term_label": "Unknown molecular function",
  "gene_symbol": "LGI1",
  "gene_name": "Leucine-rich glioma-inactivated protein 1",
  "gene": "UniProtKB:O95970"
}